{
  "term_id": "GO:0005634",
  "term_label": "nucleus",
  "gene": "UniProtKB:Q9H9E1",
  "gene_symbol": "ANKRA2",
  "gene_name": "Ankyrin repeat family A protein 2"
}